{
  "gene_name": "Zinc finger protein 626",
  "term_id": "GO:0000981",
  "term_label": "DNA-binding transcription factor activity, RNA polymerase II-specific",
  "gene": "UniProtKB:Q68DY1",
  "gene_symbol": "ZNF626"
}